{
  "gene_symbol": "CEP85",
  "gene_name": "Centrosomal protein of 85 kDa",
  "gene": "UniProtKB:Q6P2H3",
  "term_label": "Unknown molecular function",
  "term_id": "UNKNOWN:0001"
}